{
  "gene_name": "Centrin-1",
  "term_id": "GO:0000226",
  "gene_symbol": "CETN1",
  "gene": "UniProtKB:Q12798",
  "term_label": "microtubule cytoskeleton organization"
}